ATP citrate synthase activity [GO:0003878] (MF) Also known as: ATP-citrate (pro-S)-lyase activity, ATP citrate (pro-S)-lyase activity, ATP-citrate (pro-S-)-lyase activity, ATP-citric lyase activity, ATP:citrate oxaloacetate-lyase ((pro-S)-CH(2)COO(-)->acetyl-CoA) (ATP- dephosphorylating) activity, ATP:citrate oxaloacetate-lyase [(pro-S)-CH2COO-rightacetyl-CoA] (ATP-dephosphorylating), acetyl-CoA:oxaloacetate C-acetyltransferase [(pro-S)-carboxymethyl-forming, ADP-phosphorylating], acetyl-CoA:oxaloacetate acetyltransferase (isomerizing; ADP- phosphorylating) activity, acetyl-CoA:oxaloacetate acetyltransferase (isomerizing; ADP-phosphorylating), adenosine triphosphate citrate lyase activity, citrate cleavage enzyme activity, citrate-ATP lyase activity, citric cleavage enzyme activity Note: Note that this term has a MetaCyc pathway reference as the pathway only has a single step. Relationships: is a type of GO:0046912 Definition: Catalysis of the reaction: acetyl-CoA + ADP + H+ + oxaloacetate + phosphate = ATP + citrate + CoA. Regulation: regulated by regulation of ATP citrate synthase activity [GO:2000983] Sources: RHEA:21160